trans-synaptic signaling by trans-synaptic complex, modulating synaptic transmission [GO:0099557] (biological process) References: PMID:19029886 Sources: GOC:dos Relationships: is a type of trans-synaptic signaling by trans-synaptic complex [GO:0099545]; is a type of GO:0099550 Note: Note that this term was created for the SynGO project, and will be obsoleted when the SynGO annotations are made in Noctua. Definition: Cell-cell signaling between presynapse and postsynapse, mediated by transynaptic protein complexes, that modulates the synaptic transmission properties of the synapse.